{
  "gene_name": "Transgelin",
  "term_id": "UNKNOWN:0001",
  "term_label": "Unknown molecular function",
  "gene": "UniProtKB:Q01995",
  "gene_symbol": "TAGLN"
}